IgG immunoglobulin complex [GO:0071735] (CC) Sources: GOC:add, ISBN:0781765196 Definition: A protein complex composed of two identical immunoglobulin heavy chains of an IgG isotype and two identical immunoglobulin light chains, held together by disulfide bonds. An IgG immunoglobulin complex may be embedded in the plasma membrane or present in the extracellular space, in mucosal areas or other tissues, or circulating in the blood or lymph. Note: Note that an IgG immunoglobulin complex has the function of antigen binding if a suitable antigen is available. Also, IgG isotypes vary by species. Subtypes: IgG immunoglobulin complex, circulating [GO:0071736], GO:0071737 Relationships: is a type of GO:0019814 Also known as: IgG1, IgG2, IgG2a, IgG2b, IgG2c, IgG3, IgG4